5'-hydroxyl dinucleotide hydrolase activity [GO:0140432] (molecular function) Definition: Catalysis of the hydrolysis of phosphodiester bonds in 5'OH-RNA according to the reaction 5'OH-NpN-RNA + H20 = 5'OH-NpN + 5'P-RNA, where NpN represents a dinucleotide. References: PMID:31777937 Relationships: is a type of RNA exonuclease activity [GO:0004532]